{
  "gene": "UniProtKB:P61964",
  "gene_name": "WD repeat-containing protein 5",
  "term_id": "UNKNOWN:0002",
  "gene_symbol": "WDR5",
  "term_label": "Unknown biological process"
}